{
  "gene_symbol": "JARID2",
  "gene_name": "Protein Jumonji",
  "term_id": "GO:0000785",
  "gene": "UniProtKB:Q92833",
  "term_label": "chromatin"
}